{
  "term_label": "response to hypoxia",
  "gene_symbol": "VEGFB",
  "gene_name": "Vascular endothelial growth factor B",
  "gene": "UniProtKB:P49765",
  "term_id": "GO:0001666"
}